{
  "term_label": "B cell activation involved in immune response",
  "term_id": "GO:0002312",
  "gene_name": "Interferon alpha-2",
  "gene_symbol": "IFNA2",
  "gene": "UniProtKB:P01563"
}